regulation of lysosomal membrane permeability [GO:0097213] (biological process) Subtypes: GO:0097214, negative regulation of lysosomal membrane permeability [GO:0097215] Relationships: is a type of regulation of membrane permeability [GO:0090559]; is a type of lysosomal membrane organization [GO:0097212] Also known as: regulation of lysosome membrane permeability References: PMID:20544854 Sources: GOC:yaf Definition: Any process that modulates the frequency, rate or extent of the passage or uptake of molecules by the lysosomal membrane.